{
  "term_id": "UNKNOWN:0002",
  "term_label": "Unknown biological process",
  "gene_symbol": "OR51Q1",
  "gene": "UniProtKB:Q8NH59",
  "gene_name": "Olfactory receptor 51Q1"
}